{
  "gene": "UniProtKB:P48058",
  "term_label": "dendritic spine",
  "gene_name": "Glutamate receptor 4",
  "gene_symbol": "GRIA4",
  "term_id": "GO:0043197"
}